{
  "term_id": "GO:0160072",
  "term_label": "ubiquitin ligase complex scaffold activity",
  "gene": "UniProtKB:Q13617",
  "gene_name": "Cullin-2",
  "gene_symbol": "CUL2"
}